{
  "gene_name": "Membrane-associated guanylate kinase, WW and PDZ domain-containing protein 3",
  "term_id": "UNKNOWN:0001",
  "gene_symbol": "MAGI3",
  "term_label": "Unknown molecular function",
  "gene": "UniProtKB:Q5TCQ9"
}